{
  "gene": "UniProtKB:Q9UJP4",
  "gene_symbol": "KLHL21",
  "term_label": "ubiquitin-like ligase-substrate adaptor activity",
  "term_id": "GO:1990756",
  "gene_name": "Kelch-like protein 21"
}